{
  "gene_name": "Cyclin-O",
  "gene": "UniProtKB:P22674",
  "term_id": "GO:0000082",
  "term_label": "G1/S transition of mitotic cell cycle",
  "gene_symbol": "CCNO"
}